{
  "term_label": "natural killer cell mediated immunity",
  "term_id": "GO:0002228",
  "gene": "UniProtKB:Q07444",
  "gene_name": "NKG2-E type II integral membrane protein",
  "gene_symbol": "KLRC3"
}